{
  "gene_name": "Uncharacterized protein C3orf84",
  "term_label": "Unknown cellular component",
  "gene_symbol": "C3orf84",
  "gene": "UniProtKB:H3BNL1",
  "term_id": "UNKNOWN:0003"
}